{
  "term_label": "Unknown cellular component",
  "term_id": "UNKNOWN:0003",
  "gene_symbol": "DRICH1",
  "gene_name": "Aspartate-rich protein 1",
  "gene": "UniProtKB:Q6PGQ1"
}